{
  "gene_symbol": "WDR49",
  "term_id": "UNKNOWN:0001",
  "gene": "UniProtKB:Q8IV35",
  "gene_name": "WD repeat-containing protein 49",
  "term_label": "Unknown molecular function"
}